cytolysis by host of symbiont cells [GO:0051838] (biological process) Sources: GOC:add Relationships: is a type of GO:0051873 Definition: The killing by an organism of a cell in its symbiont organism by means of the rupture of cell membranes and the loss of cytoplasm. The symbiont is defined as the smaller of the organisms involved in a symbiotic interaction.